{
  "gene_symbol": "KTN1",
  "gene": "UniProtKB:Q86UP2",
  "gene_name": "Kinectin",
  "term_label": "Unknown molecular function",
  "term_id": "UNKNOWN:0001"
}